{
  "gene_symbol": "C19orf18",
  "term_id": "UNKNOWN:0002",
  "gene_name": "Uncharacterized protein C19orf18",
  "term_label": "Unknown biological process",
  "gene": "UniProtKB:Q8NEA5"
}